{
  "term_id": "UNKNOWN:0003",
  "gene_symbol": "C21orf58",
  "gene": "UniProtKB:P58505",
  "gene_name": "Uncharacterized protein C21orf58",
  "term_label": "Unknown cellular component"
}